{
  "term_id": "GO:2000311",
  "gene": "UniProtKB:Q99946",
  "term_label": "regulation of AMPA receptor activity",
  "gene_symbol": "PRRT1",
  "gene_name": "Proline-rich transmembrane protein 1"
}